{
  "term_id": "GO:0050911",
  "gene_name": "Olfactory receptor 4E1",
  "gene": "UniProtKB:P0C645",
  "term_label": "detection of chemical stimulus involved in sensory perception of smell",
  "gene_symbol": "OR4E1"
}